{
  "gene_symbol": "THUMPD3",
  "gene_name": "tRNA (guanine(6)-N2)-methyltransferase THUMP3",
  "gene": "UniProtKB:Q9BV44",
  "term_label": "tRNA (guanine) methyltransferase activity",
  "term_id": "GO:0016423"
}